{
  "gene_name": "Serine protease HTRA4",
  "gene": "UniProtKB:P83105",
  "gene_symbol": "HTRA4",
  "term_label": "positive regulation of apoptotic process",
  "term_id": "GO:0043065"
}